regulation of granzyme A production [GO:2000511] (biological process) Subtypes: negative regulation of granzyme A production [GO:2000512], positive regulation of granzyme A production [GO:2000513] Sources: GOC:obol Relationships: is a type of regulation of production of molecular mediator of immune response [GO:0002700]; regulates GO:0035746 Definition: Any process that modulates the frequency, rate or extent of granzyme A production.